pyruvate biosynthetic process from acetate [GO:0019687] (biological process) Relationships: is a type of acetate metabolic process [GO:0006083]; is a type of GO:0042866 Also known as: pyruvate anabolism from acetate, pyruvate formation from acetate, pyruvate synthesis from acetate Sources: GOC:go_curators Definition: The chemical reactions and pathways resulting in the formation of pyruvate from other compounds, including acetate.